{
  "term_id": "GO:0005634",
  "gene": "UniProtKB:Q8N3V7",
  "term_label": "nucleus",
  "gene_name": "Synaptopodin",
  "gene_symbol": "SYNPO"
}